{
  "term_label": "signal transduction",
  "gene": "UniProtKB:P34982",
  "gene_name": "Olfactory receptor 1D2",
  "gene_symbol": "OR1D2",
  "term_id": "GO:0007165"
}